{
  "term_label": "axon guidance",
  "gene_symbol": "SEMA6D",
  "term_id": "GO:0007411",
  "gene": "UniProtKB:Q8NFY4",
  "gene_name": "Semaphorin-6D"
}